{
  "term_id": "GO:0016717",
  "gene": "UniProtKB:A8MWK0",
  "gene_symbol": "FADS2B",
  "term_label": "oxidoreductase activity, acting on paired donors, with oxidation of a pair of donors resulting in the reduction of molecular oxygen to two molecules of water",
  "gene_name": "Putative fatty acid desaturase 2-like protein FADS2B"
}